{
  "term_id": "GO:0015729",
  "gene": "UniProtKB:Q9UBX3",
  "gene_symbol": "SLC25A10",
  "term_label": "oxaloacetate transport",
  "gene_name": "Mitochondrial dicarboxylate carrier"
}